{
  "gene_name": "Sodium_potassium-transporting ATPase subunit alpha-4",
  "term_label": "cell projection",
  "gene_symbol": "ATP1A4",
  "term_id": "GO:0042995",
  "gene": "UniProtKB:Q13733"
}